negative regulation of protein adenylylation [GO:1900723] (biological process) Relationships: is_a GO:0031400; is a type of regulation of protein adenylylation [GO:1900722]; negatively regulates protein adenylylation [GO:0018117] Sources: GOC:TermGenie Also known as: down regulation of protein AMPylation, down regulation of protein adenylation, down regulation of protein adenylylation, down regulation of protein amino acid adenylylation, down-regulation of protein AMPylation, down-regulation of protein adenylation, down-regulation of protein adenylylation, down-regulation of protein amino acid adenylylation, downregulation of protein AMPylation, downregulation of protein adenylation, downregulation of protein adenylylation, downregulation of protein amino acid adenylylation, inhibition of protein AMPylation, inhibition of protein adenylation, inhibition of protein amino acid adenylylation, negative regulation of protein AMPylation, negative regulation of protein adenylation, negative regulation of protein amino acid adenylylation, inhibition of protein adenylylation Definition: Any process that stops, prevents or reduces the frequency, rate or extent of protein adenylylation.